{
  "term_label": "vesicle-mediated transport",
  "gene_name": "PH and SEC7 domain-containing protein 4",
  "term_id": "GO:0016192",
  "gene": "UniProtKB:Q8NDX1",
  "gene_symbol": "PSD4"
}